{
  "term_id": "UNKNOWN:0001",
  "term_label": "Unknown molecular function",
  "gene": "UniProtKB:Q5U4P2",
  "gene_name": "Aspartate beta-hydroxylase domain-containing protein 1",
  "gene_symbol": "ASPHD1"
}